{
  "term_id": "GO:0051661",
  "gene": "UniProtKB:Q99996",
  "gene_symbol": "AKAP9",
  "gene_name": "A-kinase anchor protein 9",
  "term_label": "maintenance of centrosome location"
}